{
  "gene_name": "Retina-specific copper amine oxidase",
  "term_id": "GO:0008131",
  "gene_symbol": "AOC2",
  "term_label": "primary methylamine oxidase activity",
  "gene": "UniProtKB:O75106"
}